{
  "term_label": "regulation of microvillus assembly",
  "gene_name": "Podocalyxin",
  "gene_symbol": "PODXL",
  "gene": "UniProtKB:O00592",
  "term_id": "GO:0032534"
}